Tpg-containing telomere binding complex [GO:0043769] (cellular component) References: PMID:15353591 Definition: A complex composed of four polypeptides, a telomere-protecting terminal protein (Tpg), a telomere-associated protein (Tap), DNA polymerase (PolA) and topoisomerase I (TopA), that functions in the replication of the telomeric regions of linear chromosomes, plasmids and circular replicons of some bacterial species. Relationships: is a type of telomere cap complex [GO:0000782] Also known as: telomere complex